{
  "gene_name": "Putative protein PLEKHA9",
  "term_label": "ceramide 1-phosphate transfer activity",
  "term_id": "GO:1902388",
  "gene": "UniProtKB:O95397",
  "gene_symbol": "PLEKHA8P1"
}